{
  "gene": "UniProtKB:Q2TB90",
  "term_label": "intracellular glucose homeostasis",
  "gene_symbol": "HKDC1",
  "term_id": "GO:0001678",
  "gene_name": "Hexokinase HKDC1"
}